{
  "gene": "UniProtKB:Q9NVV4",
  "gene_symbol": "MTPAP",
  "gene_name": "Poly(A) RNA polymerase, mitochondrial",
  "term_label": "RNA 3'-end processing",
  "term_id": "GO:0031123"
}